{
  "term_label": "fascia adherens",
  "gene": "UniProtKB:Q9UI47",
  "gene_symbol": "CTNNA3",
  "term_id": "GO:0005916",
  "gene_name": "Catenin alpha-3"
}